spindle envelope [GO:0070732] (cellular component) Relationships: is_a GO:0031967 Definition: An organelle envelope that surrounds the chromosomes and the central part of the spindle apparatus during mitosis and meiosis; observed in many invertebrates. The spindle envelope consists of membrane layers, called parafusorial membranes, derived from endoplasmic reticulum membrane; in male meiosis it forms during prometaphase and persists until early in the ensuing interphase. References: PMID:19417004, PMID:6428889 Sources: GOC:mah, GOC:sart